meiotic sister chromatid arm separation [GO:0051755] (biological process) Definition: The cell cycle process in which sister chromatid arms are physically detached from each other during meiosis. Sources: GOC:ai Relationships: is a type of meiotic cell cycle process [GO:1903046]; is part of meiosis I [GO:0007127]; is part of GO:0051757 Regulation: positively regulated by GO:0062041